{
  "term_label": "protein ubiquitination",
  "gene": "UniProtKB:E7ERA6",
  "gene_symbol": "RNF223",
  "term_id": "GO:0016567",
  "gene_name": "RING finger protein 223"
}